{
  "gene_name": "Acyl-coenzyme A thioesterase 6",
  "gene_symbol": "ACOT6",
  "term_id": "GO:0006631",
  "term_label": "fatty acid metabolic process",
  "gene": "UniProtKB:Q3I5F7"
}